deoxyribonuclease (pyrimidine dimer) activity [GO:0033892] (molecular function) Relationships: is a type of DNA endonuclease activity [GO:0004520]; is a type of hydrolase activity, acting on ester bonds [GO:0016788] Definition: Catalysis of the endonucleolytic cleavage near pyrimidine dimers to products with 5'-phosphate. Sources: EC:3.1.25.1 Also known as: T4 endonuclease V activity, bacteriophage T4 endodeoxyribonuclease V activity, endodeoxyribonuclease (pyrimidine dimer) activity